{
  "term_id": "GO:0051117",
  "gene_name": "V-type proton ATPase 116 kDa subunit a 3",
  "gene_symbol": "TCIRG1",
  "gene": "UniProtKB:Q13488",
  "term_label": "ATPase binding"
}